positive regulation of cell morphogenesis [GO:0010770] (biological process) Sources: GOC:dph, GOC:tb Subtypes: positive regulation of dendrite morphogenesis [GO:0050775], GO:0051512, positive regulation of formation of radial glial scaffolds [GO:0061926], positive regulation of platelet formation [GO:1905221] Relationships: is a type of positive regulation of cell development [GO:0010720]; is a type of regulation of cell morphogenesis [GO:0022604]; positively regulates cell morphogenesis [GO:0000902] Definition: Any process that increases the frequency, rate or extent of cell morphogenesis contributing to cell differentiation. Cell morphogenesis involved in differentiation is the change in form (cell shape and size) that occurs when relatively unspecialized cells acquire specialized structural and/or functional features that characterize the cells, tissues, or organs of the mature organism or some other relatively stable phase of the organism's life history.